{
  "term_label": "protein-macromolecule adaptor activity",
  "gene_symbol": "GRB14",
  "gene_name": "Growth factor receptor-bound protein 14",
  "term_id": "GO:0030674",
  "gene": "UniProtKB:Q14449"
}